NuRD complex binding [GO:0120325] (MF) Definition: Binding to a NuRD complex. References: PMID:25150861 Sources: GOC:krc, GOC:lb Relationships: is a type of protein-containing complex binding [GO:0044877]